{
  "gene_name": "C-X-C motif chemokine 11",
  "gene": "UniProtKB:O14625",
  "gene_symbol": "CXCL11",
  "term_label": "Unknown biological process",
  "term_id": "UNKNOWN:0002"
}